aortic smooth muscle cell differentiation [GO:0035887] (biological process) Regulation: regulated by regulation of aortic smooth muscle cell differentiation [GO:1904829]; negatively regulated by negative regulation of aortic smooth muscle cell differentiation [GO:1904830]; positively regulated by positive regulation of aortic smooth muscle cell differentiation [GO:1904831] Sources: GOC:sl Definition: The process in which a relatively unspecialized cell acquires specialized features of a smooth muscle cell surrounding the aorta. Relationships: is a type of vascular associated smooth muscle cell differentiation [GO:0035886]